regulation of autophagic cell death [GO:1904092] (biological process) Definition: Any process that modulates the frequency, rate or extent of autophagic cell death. Also known as: regulation of autophagic death, regulation of programmed cell death by autophagy, regulation of programmed cell death by macroautophagy, regulation of type II programmed cell death References: PMID:25736836 Sources: GOC:TermGenie, GOC:bhm, GO_REF:0000058 Subtypes: negative regulation of autophagic cell death [GO:1904093], positive regulation of autophagic cell death [GO:1904094] Relationships: is a type of regulation of programmed cell death [GO:0043067]; regulates autophagic cell death [GO:0048102]